{
  "gene_name": "Zinc transporter 7",
  "gene": "UniProtKB:Q8NEW0",
  "gene_symbol": "SLC30A7",
  "term_label": "zinc ion import into Golgi lumen",
  "term_id": "GO:1904257"
}